regulation of blood circulation [GO:1903522] (BP) Subtypes: GO:0008016, GO:0019229, regulation of cerebral blood circulation [GO:0120276], negative regulation of blood circulation [GO:1903523], positive regulation of blood circulation [GO:1903524], regulation of gastric mucosal blood circulation [GO:1904344] References: PMID:10659969 Sources: GOC:TermGenie, GOC:mr, GO_REF:0000058 Relationships: is a type of regulation of system process [GO:0044057]; regulates GO:0008015 Also known as: regulation of hemolymph circulation Definition: Any process that modulates the frequency, rate or extent of blood circulation.